{
  "term_label": "nucleus",
  "gene_name": "Zinc finger protein 786",
  "term_id": "GO:0005634",
  "gene": "UniProtKB:Q8N393",
  "gene_symbol": "ZNF786"
}